{
  "gene_symbol": "SLC2A10",
  "term_id": "GO:1904659",
  "gene_name": "Solute carrier family 2, facilitated glucose transporter member 10",
  "gene": "UniProtKB:O95528",
  "term_label": "D-glucose transmembrane transport"
}